{
  "gene_symbol": "TCP11",
  "gene": "UniProtKB:Q8WWU5",
  "term_label": "Unknown molecular function",
  "term_id": "UNKNOWN:0001",
  "gene_name": "T-complex protein 11 homolog"
}